{
  "gene": "UniProtKB:P0C7V8",
  "term_label": "Unknown biological process",
  "gene_symbol": "DCAF8L2",
  "gene_name": "DDB1- and CUL4-associated factor 8-like protein 2",
  "term_id": "UNKNOWN:0002"
}